positive regulation of T-helper 2 cell differentiation [GO:0045630] (biological process) Note: Note that immunologists typically use the word 'development' to refer to cells of B or T cell lineages undergoing the process that GO describes as 'cell differentiation'. Also known as: up regulation of T-helper 2 cell differentiation, up-regulation of T-helper 2 cell differentiation, upregulation of T-helper 2 cell differentiation, activation of T-helper 2 cell differentiation, stimulation of T-helper 2 cell differentiation, positive regulation of T-helper 2 cell development Relationships: is a type of positive regulation of type 2 immune response [GO:0002830]; is a type of positive regulation of T-helper cell differentiation [GO:0045624]; is a type of regulation of T-helper 2 cell differentiation [GO:0045628]; positively regulates T-helper 2 cell differentiation [GO:0045064] Sources: GOC:go_curators Definition: Any process that activates or increases the frequency, rate or extent of T-helper 2 cell differentiation.